{
  "gene_name": "Transmembrane glycoprotein NMB",
  "gene": "UniProtKB:Q14956",
  "term_label": "integrin binding",
  "gene_symbol": "GPNMB",
  "term_id": "GO:0005178"
}